{
  "gene_symbol": "FTO",
  "gene": "UniProtKB:Q9C0B1",
  "term_id": "GO:0042245",
  "term_label": "RNA repair",
  "gene_name": "Alpha-ketoglutarate-dependent dioxygenase FTO"
}